{
  "term_label": "retrograde transport, endosome to Golgi",
  "gene": "UniProtKB:Q9NW61",
  "gene_name": "Pleckstrin homology domain-containing family J member 1",
  "term_id": "GO:0042147",
  "gene_symbol": "PLEKHJ1"
}